regulation of cell proliferation in midbrain [GO:1904933] (biological process) Subtypes: negative regulation of cell proliferation in midbrain [GO:1904934], GO:1904935 References: PMID:18953410, PMID:24431302 Sources: GOC:PARL, GOC:TermGenie, GOC:bf, GO_REF:0000058 Relationships: is a type of GO:2000177; RO_0002211 cell proliferation in midbrain [GO:0033278] Definition: Any process that modulates the frequency, rate or extent of cell proliferation in midbrain. Also known as: regulation of cell proliferation in mesencephalon, regulation of mesencepahalic cell proliferation